{
  "term_label": "pyrimidine nucleotide transmembrane transporter activity",
  "gene_symbol": "SLC25A33",
  "term_id": "GO:0015218",
  "gene_name": "Solute carrier family 25 member 33",
  "gene": "UniProtKB:Q9BSK2"
}